{
  "term_label": "serine-type endopeptidase inhibitor activity",
  "term_id": "GO:0004867",
  "gene": "UniProtKB:Q6UXR4",
  "gene_symbol": "SERPINA13P",
  "gene_name": "Putative serpin A13"
}